positive regulation of Wnt signaling pathway, planar cell polarity pathway [GO:2000096] (biological process) Definition: Any process that activates or increases the frequency, rate or extent of Wnt signaling pathway, planar cell polarity pathway. Sources: GOC:BHF Also known as: positive regulation of PCP pathway, positive regulation of Wnt receptor signaling pathway, planar cell polarity pathway, positive regulation of Wnt receptor signalling pathway, planar cell polarity pathway, positive regulation of Wnt-activated signaling pathway, planar cell polarity pathway, positive regulation of Wnt-JNK signaling pathway, positive regulation of Wnt-PCP signaling pathway, positive regulation of non-canonical Wnt signaling pathway Relationships: is a type of positive regulation of non-canonical Wnt signaling pathway [GO:2000052]; is a type of regulation of Wnt signaling pathway, planar cell polarity pathway [GO:2000095]; positively regulates GO:0060071